{
  "term_id": "GO:0098609",
  "gene_name": "Disks large homolog 1",
  "gene_symbol": "DLG1",
  "term_label": "cell-cell adhesion",
  "gene": "UniProtKB:Q12959"
}